{
  "term_id": "GO:0005634",
  "gene": "UniProtKB:P35680",
  "term_label": "nucleus",
  "gene_symbol": "HNF1B",
  "gene_name": "Hepatocyte nuclear factor 1-beta"
}